alpha7-beta1 integrin-nicotinamide riboside kinase complex [GO:0071119] (cellular component) References: PMID:12941630 Definition: A protein complex that consists of an alpha7-beta1 integrin complex bound to nicotinamide riboside kinase 2 (also known as muscle integrin binding protein, MIBP). Also known as: ITGA7-ITGB1-ITGB1BP3 complex Relationships: is a type of plasma membrane protein complex [GO:0098797]